negative regulation of androstenedione secretion [GO:2000838] (biological process) Definition: Any process that stops, prevents or reduces the frequency, rate or extent of androstenedione secretion. Also known as: negative regulation of androst-4-ene-3,17-dione secretion Sources: GOC:sl Relationships: is a type of GO:0032369; is a type of negative regulation of hormone secretion [GO:0046888]; is a type of regulation of androstenedione secretion [GO:2000837]; negatively regulates androstenedione secretion [GO:0035941]